{
  "term_id": "GO:0005634",
  "gene": "UniProtKB:O95600",
  "term_label": "nucleus",
  "gene_name": "Krueppel-like factor 8",
  "gene_symbol": "KLF8"
}